{
  "gene_name": "Transmembrane emp24 domain-containing protein 6",
  "gene_symbol": "TMED6",
  "term_id": "UNKNOWN:0001",
  "term_label": "Unknown molecular function",
  "gene": "UniProtKB:Q8WW62"
}